{
  "term_id": "GO:0004713",
  "gene": "UniProtKB:P0C1S8",
  "term_label": "protein tyrosine kinase activity",
  "gene_name": "Wee1-like protein kinase 2",
  "gene_symbol": "WEE2"
}